positive regulation of neutrophil mediated killing of fungus [GO:0070965] (biological process) Relationships: is a type of GO:0070953; is a type of positive regulation of neutrophil mediated killing of symbiont cell [GO:0070961]; positively regulates neutrophil-mediated killing of fungus [GO:0070947] Also known as: up regulation of neutrophil mediated killing of fungus, up-regulation of neutrophil mediated killing of fungus, upregulation of neutrophil mediated killing of fungus, activation of neutrophil mediated killing of fungus, stimulation of neutrophil mediated killing of fungus Sources: GOC:add, GOC:mah Definition: Any process that increases the frequency, rate or extent of the directed killing of a fungal cell by a neutrophil.